positive regulation of hippocampal neuron apoptotic process [GO:0110090] (biological process) Relationships: is a type of positive regulation of neuron apoptotic process [GO:0043525]; is a type of regulation of hippocampal neuron apoptotic process [GO:0110089]; positively regulates hippocampal neuron apoptotic process [GO:0110088] References: PMID:18940801 Sources: GOC:sl Definition: Any process that activates or increases the frequency, rate or extent of cell death by apoptotic process in hippocampal neurons.